{
  "gene_symbol": "AP4M1",
  "gene": "UniProtKB:O00189",
  "term_label": "protein targeting",
  "gene_name": "AP-4 complex subunit mu-1",
  "term_id": "GO:0006605"
}